ferrous iron transmembrane transporter activity [GO:0015093] (MF) Subtypes: GO:0061840 Sources: ISBN:0198506732 Relationships: is a type of GO:0005381 Definition: Enables the transfer of ferrous iron (Fe(II) or Fe2+) ions from one side of a membrane to the other. Also known as: ferrous iron uptake transmembrane transporter activity